{
  "gene_symbol": "NPPB",
  "gene": "UniProtKB:P16860",
  "gene_name": "Natriuretic peptides B",
  "term_label": "negative regulation of systemic arterial blood pressure",
  "term_id": "GO:0003085"
}